tridecane biosynthetic process [GO:1900632] (biological process) Definition: The chemical reactions and pathways resulting in the formation of tridecane. Sources: GOC:TermGenie, GOC:mengo_curators Also known as: tridecane anabolism, tridecane biosynthesis, tridecane formation, tridecane synthesis Relationships: is a type of alkane biosynthetic process [GO:0043447]; is a type of tridecane metabolic process [GO:1900631] Regulation: regulated by GO:1900884; negatively regulated by negative regulation of tridecane biosynthetic process [GO:1900885]; RO_0002213 by positive regulation of tridecane biosynthetic process [GO:1900886]